plasma cell differentiation [GO:0002317] (biological process) Also known as: plasma cell development Note: Note that immunologists typically use the word 'development' to refer to cells of B or T cell lineages undergoing the process that GO describes as 'cell differentiation'. Relationships: is a type of mature B cell differentiation involved in immune response [GO:0002313] Regulation: regulated by GO:1900098; negatively regulated by negative regulation of plasma cell differentiation [GO:1900099]; RO_0002213 by positive regulation of plasma cell differentiation [GO:1900100] Sources: GOC:jal Definition: The process in which a B cell acquires the specialized features of a plasma cell. A plasma cell is a lymphocyte which develops from a B cell and produces high amounts of antibody.